{
  "gene_name": "NXPE family member 1",
  "gene": "UniProtKB:Q8N323",
  "gene_symbol": "NXPE1",
  "term_id": "UNKNOWN:0003",
  "term_label": "Unknown cellular component"
}